{
  "gene_symbol": "NCALD",
  "term_label": "calcium-mediated signaling",
  "gene_name": "Neurocalcin-delta",
  "term_id": "GO:0019722",
  "gene": "UniProtKB:P61601"
}